{
  "gene_name": "Glycerol-3-phosphate dehydrogenase, mitochondrial",
  "gene": "UniProtKB:P43304",
  "term_label": "glycerol-3-phosphate metabolic process",
  "gene_symbol": "GPD2",
  "term_id": "GO:0006072"
}